{
  "gene_name": "T cell receptor beta variable 7-6",
  "gene_symbol": "TRBV7-6",
  "term_label": "cell surface receptor signaling pathway",
  "term_id": "GO:0007166",
  "gene": "UniProtKB:A0A1B0GX31"
}